{
  "term_id": "GO:0005788",
  "gene_name": "Endoplasmic reticulum chaperone BiP",
  "term_label": "endoplasmic reticulum lumen",
  "gene_symbol": "HSPA5",
  "gene": "UniProtKB:P11021"
}